{
  "gene": "UniProtKB:Q8NCM2",
  "term_id": "GO:0071805",
  "gene_name": "Potassium voltage-gated channel subfamily H member 5",
  "term_label": "potassium ion transmembrane transport",
  "gene_symbol": "KCNH5"
}